{
  "term_label": "TRAPP complex",
  "gene_name": "Trafficking protein particle complex subunit 2",
  "gene": "UniProtKB:P0DI81",
  "term_id": "GO:0030008",
  "gene_symbol": "TRAPPC2"
}